transforming growth factor beta receptor activity, type I [GO:0005025] (molecular function) Sources: GOC:mah Relationships: is a type of transforming growth factor beta receptor activity [GO:0005024] Also known as: type I TGF-beta receptor activity, type I TGFbeta receptor activity, type I transforming growth factor beta receptor activity, transforming growth factor beta ligand binding to type I receptor Definition: Combining with a complex of transforming growth factor beta and a type II TGF-beta receptor to initiate a change in cell activity; upon binding, acts as a downstream transducer of TGF-beta signals.